{
  "gene_name": "Protein FAM117A",
  "gene_symbol": "FAM117A",
  "gene": "UniProtKB:Q9C073",
  "term_id": "UNKNOWN:0003",
  "term_label": "Unknown cellular component"
}